{
  "gene_name": "Ribosomal protein S6 kinase beta-2",
  "term_label": "TORC1 signaling",
  "gene": "UniProtKB:Q9UBS0",
  "term_id": "GO:0038202",
  "gene_symbol": "RPS6KB2"
}